{
  "term_label": "nuclear envelope",
  "gene_name": "BCL2_adenovirus E1B 19 kDa protein-interacting protein 3",
  "gene": "UniProtKB:Q12983",
  "gene_symbol": "BNIP3",
  "term_id": "GO:0005635"
}